{
  "term_id": "GO:0009897",
  "gene_symbol": "CD28",
  "gene": "UniProtKB:P10747",
  "term_label": "external side of plasma membrane",
  "gene_name": "T-cell-specific surface glycoprotein CD28"
}